S phase [GO:0051320] (biological process) Definition: The cell cycle phase, following G1, during which DNA synthesis takes place. Also known as: S-phase Sources: GOC:mtg_cell_cycle Subtypes: mitotic S phase [GO:0000084], meiotic S phase [GO:0051332] Relationships: is a type of cell cycle phase [GO:0022403]; is part of interphase [GO:0051325] Note: Note that this term should not be used for direct annotation. If you are trying to make an annotation to x phase, it is likely that the correct annotation is 'regulation of x/y phase transition' or to a process which occurs during the reported phase (i.e mitotic DNA replication for mitotic S-phase). To capture the phase when a specific location or process is observed, the phase term can be used in an annotation extension (PMID:24885854) applied to a cellular component term (with the relation exists_during) or a biological process term (with the relation happens_during).